GTP:coenzyme F420 guanyltransferase activity [GO:0052754] (molecular function) Relationships: is a type of guanylyltransferase activity [GO:0070568] Definition: Catalysis of the reaction: GTP + factor gamma-F420-2 + H+ = coenzyme F390-G + diphosphate. Sources: GOC:mengo_curators, MetaCyc:RXN-18273 Also known as: GTP:coenzyme F420 guanylyltransferase activity, coenzyme F390-G synthetase activity